{
  "gene_symbol": "CMPK1",
  "gene_name": "UMP-CMP kinase",
  "term_label": "nucleus",
  "gene": "UniProtKB:P30085",
  "term_id": "GO:0005634"
}